{
  "gene": "UniProtKB:A4D1P6",
  "term_id": "GO:0045022",
  "gene_name": "WD repeat-containing protein 91",
  "term_label": "early endosome to late endosome transport",
  "gene_symbol": "WDR91"
}